{
  "gene_name": "Olfactory receptor 2W1",
  "term_id": "GO:0005886",
  "term_label": "plasma membrane",
  "gene": "UniProtKB:Q9Y3N9",
  "gene_symbol": "OR2W1"
}